{
  "gene_name": "6-phosphofructo-2-kinase_fructose-2,6-bisphosphatase 2",
  "term_label": "fructose-2,6-bisphosphate 2-phosphatase activity",
  "term_id": "GO:0004331",
  "gene_symbol": "PFKFB2",
  "gene": "UniProtKB:O60825"
}